nucleomorph [GO:0033009] (cellular component) Definition: A small, vestigial nucleus found in some plastids that derive from a eukaryotic endosymbiont. Observed in chlorarachniophytes and cryptomonads, which acquired their plastids from a green and red alga respectively. Relationships: is a type of intracellular membrane-bounded organelle [GO:0043231]; is part of GO:0009536 References: PMID:16760254